{
  "gene_symbol": "SLFN14",
  "gene_name": "Protein SLFN14",
  "term_id": "GO:0006402",
  "term_label": "mRNA catabolic process",
  "gene": "UniProtKB:P0C7P3"
}